{
  "term_label": "kinase binding",
  "gene_symbol": "MYOM1",
  "gene": "UniProtKB:P52179",
  "gene_name": "Myomesin-1",
  "term_id": "GO:0019900"
}